gap junction channel activity involved in cardiac conduction electrical coupling [GO:0086075] (molecular function) Definition: A wide pore channel activity that enables a direct cytoplasmic connection from one cardiomyocyte to an adjacent cardiomyocyte. The gap junction passes electrical signals between the cells contributing to cardiac conduction. Subtypes: gap junction channel activity involved in SA node cell-atrial cardiac muscle cell electrical coupling [GO:0086020], gap junction channel activity involved in atrial cardiac muscle cell-AV node cell electrical coupling [GO:0086076], gap junction channel activity involved in AV node cell-bundle of His cell electrical coupling [GO:0086077], gap junction channel activity involved in bundle of His cell-Purkinje myocyte electrical coupling [GO:0086078], GO:0086079 Sources: GOC:BHF, GOC:mtg_cardiac_conduct_nov11 Relationships: is a type of gap junction channel activity involved in cell communication by electrical coupling [GO:1903763]; is part of GO:0086064